mitochondrial guanine nucleotide transmembrane transport [GO:0140140] (biological process) Relationships: is a type of guanine transmembrane transport [GO:1903716] Definition: The process in which a guanine nucleotide is transported across a mitochondrial membrane, into or out of the mitochondrion. References: PMID:14998997 Sources: GOC:vw